{
  "term_label": "replication fork processing",
  "gene_name": "E3 ubiquitin-protein ligase RFWD3",
  "gene": "UniProtKB:Q6PCD5",
  "gene_symbol": "RFWD3",
  "term_id": "GO:0031297"
}